{
  "term_id": "GO:0005892",
  "term_label": "acetylcholine-gated channel complex",
  "gene": "UniProtKB:P11230",
  "gene_symbol": "CHRNB1",
  "gene_name": "Acetylcholine receptor subunit beta"
}